alcohol catabolic process [GO:0046164] (biological process) Regulation: regulated by regulation of alcohol catabolic process [GO:1900419]; negatively regulated by negative regulation of alcohol catabolic process [GO:1900420]; RO_0002213 by positive regulation of alcohol catabolic process [GO:1900421] Definition: The chemical reactions and pathways resulting in the breakdown of alcohols, any of a class of compounds containing one or more hydroxyl groups attached to a saturated carbon atom. Sources: GOC:ai Also known as: alcohol breakdown, alcohol catabolism, alcohol degradation Relationships: is a type of alcohol metabolic process [GO:0006066]; is a type of small molecule catabolic process [GO:0044282] Subtypes: GO:0006707, ecdysone catabolic process [GO:0006708], prenol catabolic process [GO:0016092], polyprenol catabolic process [GO:0016095], GO:0019622, cyclopentanol catabolic process [GO:0033022], primary alcohol catabolic process [GO:0034310], GO:0045150, rhodopsin catabolic process [GO:0046155], polyol catabolic process [GO:0046174], octopamine catabolic process [GO:0046334], abscisic acid catabolic process [GO:0046345], GO:1900580, fonsecin catabolic process [GO:1900768], tetracenomycin C catabolic process [GO:1901105], monensin A catabolic process [GO:1901729], vitamin D3 catabolic process [GO:1901754], GO:1902049, GO:1902245, fatty alcohol catabolic process [GO:1903174]